phosphoribosyl-ATP diphosphatase activity [GO:0004636] (molecular function) Sources: EC:3.6.1.31, RHEA:22828 Definition: Catalysis of the reaction: 1-(5-phospho-D-ribosyl)-ATP + H2O = 1-(5-phosphonatoribosyl)-5'-AMP + diphosphate + H+. Relationships: is a type of pyrophosphatase activity [GO:0016462] Also known as: phosphoribosyl-ATP pyrophosphatase activity, 1-(5-phosphoribosyl)-ATP diphosphohydrolase activity, phosphoribosyladenosine triphosphate pyrophosphatase activity